{
  "gene": "UniProtKB:P03952",
  "gene_symbol": "KLKB1",
  "gene_name": "Plasma kallikrein",
  "term_id": "GO:0031639",
  "term_label": "plasminogen activation"
}